malonyl-CoA synthetase activity [GO:0090409] (molecular function) Definition: Catalysis of the reaction: malonate + ATP + coenzyme A = malonyl-CoA + AMP + diphosphate. Sources: RHEA:32139 Relationships: is a type of GO:0016405